{
  "gene_symbol": "GABRA6",
  "term_label": "postsynapse",
  "gene_name": "Gamma-aminobutyric acid receptor subunit alpha-6",
  "gene": "UniProtKB:Q16445",
  "term_id": "GO:0098794"
}